limonene-1,2-epoxide hydrolase activity [GO:0018744] (MF) Also known as: limonene oxide hydrolase activity Sources: EC:3.3.2.8 Relationships: is a type of epoxide hydrolase activity [GO:0004301] Definition: Catalysis of the reaction: limonene-1,2-epoxide + H2O = limonene-1,2-diol. Other substrates include alicyclic and 1-methyl-substituted epoxides, such as 1-methylcyclohexene oxide, indene oxide and cyclohexene oxide.